{
  "gene_symbol": "GBGT1",
  "gene": "UniProtKB:Q8N5D6",
  "gene_name": "Globoside alpha-1,3-N-acetylgalactosaminyltransferase 1",
  "term_id": "GO:0047277",
  "term_label": "globoside alpha-N-acetylgalactosaminyltransferase activity"
}